{
  "gene_name": "Inactive ubiquitin carboxyl-terminal hydrolase 53",
  "gene": "UniProtKB:Q70EK8",
  "term_id": "GO:0010996",
  "term_label": "response to auditory stimulus",
  "gene_symbol": "USP53"
}